{
  "term_id": "GO:0005730",
  "gene_name": "RNA 3'-terminal phosphate cyclase-like protein",
  "gene_symbol": "RCL1",
  "gene": "UniProtKB:Q9Y2P8",
  "term_label": "nucleolus"
}